{
  "gene_symbol": "CA11",
  "gene_name": "Carbonic anhydrase-related protein 11",
  "term_id": "UNKNOWN:0002",
  "term_label": "Unknown biological process",
  "gene": "UniProtKB:O75493"
}